{
  "gene_symbol": "UBASH3B",
  "term_id": "GO:0070527",
  "gene": "UniProtKB:Q8TF42",
  "term_label": "platelet aggregation",
  "gene_name": "Ubiquitin-associated and SH3 domain-containing protein B"
}